{
  "gene": "UniProtKB:P86452",
  "term_id": "GO:0005634",
  "gene_name": "Zinc finger BED domain-containing protein 6",
  "term_label": "nucleus",
  "gene_symbol": "ZBED6"
}